{
  "term_id": "GO:0045296",
  "gene_name": "Plakophilin-2",
  "gene_symbol": "PKP2",
  "gene": "UniProtKB:Q99959",
  "term_label": "cadherin binding"
}